{
  "gene_name": "Radixin",
  "gene": "UniProtKB:P35241",
  "term_id": "GO:0003779",
  "gene_symbol": "RDX",
  "term_label": "actin binding"
}